{
  "gene_name": "Hepatocyte nuclear factor 6",
  "term_id": "GO:0006357",
  "gene": "UniProtKB:Q9UBC0",
  "gene_symbol": "ONECUT1",
  "term_label": "regulation of transcription by RNA polymerase II"
}